{
  "gene": "UniProtKB:O60673",
  "term_id": "GO:0005634",
  "gene_symbol": "REV3L",
  "gene_name": "DNA polymerase zeta catalytic subunit",
  "term_label": "nucleus"
}